{
  "term_id": "GO:0043027",
  "gene_symbol": "BIRC7",
  "gene": "UniProtKB:Q96CA5",
  "gene_name": "Baculoviral IAP repeat-containing protein 7",
  "term_label": "cysteine-type endopeptidase inhibitor activity involved in apoptotic process"
}